{
  "term_id": "GO:0060090",
  "term_label": "molecular adaptor activity",
  "gene_symbol": "CAV1",
  "gene": "UniProtKB:Q03135",
  "gene_name": "Caveolin-1"
}